{
  "term_label": "nuclear localization sequence binding",
  "gene_symbol": "NUP153",
  "gene": "UniProtKB:P49790",
  "gene_name": "Nuclear pore complex protein Nup153",
  "term_id": "GO:0008139"
}